plant-type cell wall organization [GO:0009664] (biological process) Also known as: plant-type cell wall organisation, cell wall organization and biogenesis, cellulose and pectin-containing cell wall organization and biogenesis, plant-type cell wall organization and biogenesis Sources: GOC:jid, GOC:mtg_sensu Relationships: is a type of cell wall organization [GO:0071555]; is a type of plant-type cell wall organization or biogenesis [GO:0071669] Definition: A process that results in the assembly and arrangement of constituent parts of the cellulose and pectin-containing cell wall, or in the disassembly of the cellulose and pectin-containing cell wall. This process is carried out at the cellular level. An example of this process is found in Arabidopsis thaliana. Subtypes: plant-type cell wall modification [GO:0009827], GO:0071668